{
  "gene_name": "Protein SSXT",
  "gene": "UniProtKB:Q15532",
  "gene_symbol": "SS18",
  "term_label": "transcription coactivator activity",
  "term_id": "GO:0003713"
}